{
  "gene_symbol": "HYCC1",
  "gene": "UniProtKB:Q9BYI3",
  "term_id": "GO:0046854",
  "gene_name": "Hyccin",
  "term_label": "phosphatidylinositol phosphate biosynthetic process"
}